{
  "gene": "UniProtKB:P14136",
  "term_id": "GO:0005200",
  "term_label": "structural constituent of cytoskeleton",
  "gene_symbol": "GFAP",
  "gene_name": "Glial fibrillary acidic protein"
}